positive regulation of nitric-oxide synthase activity [GO:0051000] (biological process) Sources: GOC:ai Definition: Any process that activates or increases the activity of the enzyme nitric-oxide synthase. Also known as: NOS activator, nitric-oxide synthase activator, positive regulation of NOS activity, up regulation of nitric-oxide synthase activity, up-regulation of nitric-oxide synthase activity, upregulation of nitric-oxide synthase activity, activation of nitric-oxide synthase activity, stimulation of nitric-oxide synthase activity Relationships: is_a GO:0050999; is a type of positive regulation of oxidoreductase activity [GO:0051353]; positively regulates GO:0004517